cellular response to histamine [GO:0071420] (biological process) Also known as: cellular response to histamine stimulus Sources: GOC:mah Relationships: is a type of response to histamine [GO:0034776]; is a type of GO:1901699 Definition: Any process that results in a change in state or activity of a cell (in terms of movement, secretion, enzyme production, gene expression, etc.) as a result of a histamine stimulus. Histamine, the biogenic amine 2-(1H-imidazol-4-yl)ethanamine, is involved in local immune responses as well as regulating physiological function in the gut and acting as a neurotransmitter.